{
  "gene_name": "Asialoglycoprotein receptor 2",
  "gene_symbol": "ASGR2",
  "term_id": "GO:0006955",
  "gene": "UniProtKB:P07307",
  "term_label": "immune response"
}